{
  "term_label": "protein tyrosine kinase activity",
  "gene_symbol": "AATK",
  "gene": "UniProtKB:Q6ZMQ8",
  "gene_name": "Serine_threonine-protein kinase LMTK1",
  "term_id": "GO:0004713"
}